{
  "gene_name": "AP-5 complex subunit beta-1",
  "gene_symbol": "AP5B1",
  "gene": "UniProtKB:Q2VPB7",
  "term_label": "AP-type membrane coat adaptor complex",
  "term_id": "GO:0030119"
}